{
  "term_id": "GO:0006357",
  "gene": "UniProtKB:Q9C0A1",
  "term_label": "regulation of transcription by RNA polymerase II",
  "gene_symbol": "ZFHX2",
  "gene_name": "Zinc finger homeobox protein 2"
}